{
  "gene": "UniProtKB:P09874",
  "term_id": "GO:0140806",
  "gene_name": "Poly [ADP-ribose] polymerase 1",
  "gene_symbol": "PARP1",
  "term_label": "NAD+-protein-aspartate ADP-ribosyltransferase activity"
}